{
  "gene_name": "Intelectin-1",
  "term_id": "UNKNOWN:0002",
  "term_label": "Unknown biological process",
  "gene": "UniProtKB:Q8WWA0",
  "gene_symbol": "ITLN1"
}